{
  "gene_name": "Voltage-dependent calcium channel gamma-5 subunit",
  "term_id": "GO:0016247",
  "gene_symbol": "CACNG5",
  "term_label": "channel regulator activity",
  "gene": "UniProtKB:Q9UF02"
}